{
  "gene_name": "Spastin",
  "term_label": "spindle",
  "gene_symbol": "SPAST",
  "term_id": "GO:0005819",
  "gene": "UniProtKB:Q9UBP0"
}